epithelial cell differentiation involved in embryonic placenta development [GO:0060671] (biological process) Relationships: is a type of epithelial cell differentiation [GO:0030855]; is a type of cell differentiation involved in embryonic placenta development [GO:0060706]; BFO_0000050 labyrinthine layer development [GO:0060711] Definition: The process in which a trophoblast cell acquires specialized features of an epithelial cell of the placental labyrinthine layer. References: PMID:16916377 Sources: GOC:dph